{
  "term_id": "GO:0032367",
  "gene": "UniProtKB:P61916",
  "gene_name": "NPC intracellular cholesterol transporter 2",
  "term_label": "intracellular cholesterol transport",
  "gene_symbol": "NPC2"
}